{
  "term_id": "GO:0019789",
  "gene": "UniProtKB:P29590",
  "gene_symbol": "PML",
  "gene_name": "Protein PML",
  "term_label": "SUMO transferase activity"
}